negative regulation of mammary stem cell proliferation [GO:2000102] (biological process) Relationships: is a type of GO:0008285; is a type of GO:0051093; is a type of GO:0051241; is a type of GO:2000101; negatively regulates mammary stem cell proliferation [GO:0002174] Sources: GOC:obol Definition: Any process that stops, prevents, or reduces the frequency, rate or extent of mammary stem cell proliferation.